siderophore catabolic process [GO:0046215] (BP) Subtypes: pyoverdine catabolic process [GO:0002050], GO:0042859, achromobactin catabolic process [GO:0042862], GO:0042865, GO:0046214 Relationships: is_a siderophore metabolic process [GO:0009237]; is a type of secondary metabolite catabolic process [GO:0090487] Also known as: siderophore breakdown, siderophore catabolism, siderophore degradation, siderochrome catabolism Sources: GOC:ai Definition: The chemical reactions and pathways resulting in the breakdown of siderophores, low molecular weight Fe(III)-chelating substances made by aerobic or facultatively anaerobic bacteria, especially when growing under iron deficient conditions. The complexes of Fe(3+)-siderophores have very high stability constants and are taken up by specific transport systems by microorganisms; the subsequent release of iron requires enzymatic action.